mandelate metabolic process [GO:0018924] (biological process) Definition: The chemical reactions and pathways involving mandelate, the anion of mandelic acid. Mandelic acid (alpha-hydroxybenzeneacetic acid) is an 8-carbon alpha-hydroxy acid (AHA) that is used in organic chemistry and as a urinary antiseptic. Subtypes: mandelate catabolic process [GO:0019596], mandelate biosynthetic process [GO:0046236] Relationships: is a type of monocarboxylic acid metabolic process [GO:0032787]; is a type of GO:0042537 Sources: GOC:jl Also known as: mandelate metabolism, mandelic acid metabolic process, mandelic acid metabolism